{
  "term_label": "protein localization to heterochromatin",
  "term_id": "GO:0097355",
  "gene": "UniProtKB:Q9UK61",
  "gene_name": "Protein TASOR",
  "gene_symbol": "TASOR"
}